{
  "gene_symbol": "TMEM41A",
  "gene": "UniProtKB:Q96HV5",
  "term_id": "UNKNOWN:0003",
  "gene_name": "Transmembrane protein 41A",
  "term_label": "Unknown cellular component"
}